asexual spore wall [GO:0097515] (cellular component) Definition: A specialized envelope lying outside the cell membrane of a spore derived from an asexual process. Examples of this process are found in bacterial and fungal species. Sources: GOC:cjm, GOC:mah Relationships: is a type of spore wall [GO:0031160]